{
  "gene": "UniProtKB:Q6ZRP0",
  "term_id": "UNKNOWN:0001",
  "gene_name": "Proline-rich protein 23C",
  "gene_symbol": "PRR23C",
  "term_label": "Unknown molecular function"
}